anterior midgut invagination [GO:0007375] (biological process) Definition: Internalization of the anterior midgut into the interior of the embryo. Relationships: is a type of morphogenesis of embryonic epithelium [GO:0016331]; is part of GO:0010004 Sources: ISBN:0879694238